{
  "gene": "UniProtKB:D6RGH6",
  "term_label": "regulation of DNA-templated DNA replication initiation",
  "gene_name": "Multicilin",
  "gene_symbol": "MCIDAS",
  "term_id": "GO:0030174"
}